{
  "term_label": "brush border membrane",
  "gene": "UniProtKB:Q14728",
  "gene_name": "Major facilitator superfamily domain-containing protein 10",
  "term_id": "GO:0031526",
  "gene_symbol": "MFSD10"
}